{
  "gene_name": "Endothelin-3",
  "gene_symbol": "EDN3",
  "term_label": "endothelin B receptor binding",
  "gene": "UniProtKB:P14138",
  "term_id": "GO:0031708"
}